activin receptor binding [GO:0070697] (molecular function) Sources: GOC:BHF, GOC:vk Subtypes: type I activin receptor binding [GO:0070698], type II activin receptor binding [GO:0070699] Relationships: is a type of transmembrane receptor protein serine/threonine kinase binding [GO:0070696] Definition: Binding to an activin receptor.